{
  "gene_name": "Hamartin",
  "term_label": "Unknown molecular function",
  "term_id": "UNKNOWN:0001",
  "gene_symbol": "TSC1",
  "gene": "UniProtKB:Q92574"
}